{
  "gene": "UniProtKB:Q9UQF0",
  "gene_symbol": "ERVW-1",
  "term_label": "syncytium formation by plasma membrane fusion",
  "gene_name": "Syncytin-1",
  "term_id": "GO:0000768"
}